{
  "gene": "UniProtKB:Q99988",
  "term_id": "GO:0160144",
  "gene_symbol": "GDF15",
  "gene_name": "Growth_differentiation factor 15",
  "term_label": "GDF15-GFRAL signaling pathway"
}